{
  "term_label": "Unknown cellular component",
  "gene_symbol": "GPX6",
  "gene": "UniProtKB:P59796",
  "gene_name": "Glutathione peroxidase 6",
  "term_id": "UNKNOWN:0003"
}